{
  "gene_name": "Kinesin-like protein KIF3C",
  "term_label": "microtubule binding",
  "gene": "UniProtKB:O14782",
  "gene_symbol": "KIF3C",
  "term_id": "GO:0008017"
}